xyloglucan metabolic process [GO:0010411] (biological process) Sources: GOC:tair_curators Definition: The chemical reactions and pathways involving xyloglucan, the cross-linking glycan composed of (1->4)-beta-D-glucan backbone substituted at regular intervals with beta-D-xylosyl-(1->6) residues, which is present in the primary cell wall of most higher plants. Subtypes: xyloglucan biosynthetic process [GO:0009969], xyloglucan catabolic process [GO:2000899] Relationships: is a type of GO:0044042 Also known as: xyloglucan metabolism